{
  "gene": "UniProtKB:A2A3K4",
  "term_id": "GO:0004725",
  "gene_symbol": "PTPDC1",
  "gene_name": "Protein tyrosine phosphatase domain-containing protein 1",
  "term_label": "protein tyrosine phosphatase activity"
}